{
  "gene_name": "Small conductance calcium-activated potassium channel protein 3",
  "term_label": "calmodulin binding",
  "gene": "UniProtKB:Q9UGI6",
  "gene_symbol": "KCNN3",
  "term_id": "GO:0005516"
}